{
  "gene_name": "COP9 signalosome complex subunit 6",
  "term_id": "GO:0008180",
  "gene": "UniProtKB:Q7L5N1",
  "term_label": "COP9 signalosome",
  "gene_symbol": "COPS6"
}